positive regulation of basophil degranulation [GO:1903583] (BP) Definition: Any process that activates or increases the frequency, rate or extent of basophil degranulation. Also known as: up regulation of basophil degranulation, up-regulation of basophil degranulation, upregulation of basophil degranulation, activation of basophil degranulation References: PMID:10880837 Sources: GOC:TermGenie, GO_REF:0000058 Relationships: is a type of positive regulation of myeloid leukocyte mediated immunity [GO:0002888]; is a type of positive regulation of leukocyte degranulation [GO:0043302]; is a type of GO:0050778; is a type of regulation of basophil degranulation [GO:1903581]; positively regulates basophil degranulation [GO:0002561]